{
  "gene_name": "Fibroblast growth factor receptor 2",
  "gene": "UniProtKB:P21802",
  "term_label": "positive regulation of cell population proliferation",
  "term_id": "GO:0008284",
  "gene_symbol": "FGFR2"
}